cellodextrin phosphorylase activity [GO:0050102] (molecular function) Relationships: is a type of hexosyltransferase activity [GO:0016758] Also known as: 1,4-beta-D-oligo-D-glucan:phosphate alpha-D-glucosyltransferase activity, beta-1,4-oligoglucan:orthophosphate glucosyltransferase activity Sources: EC:2.4.1.49, MetaCyc:CELLODEXTRIN-PHOSPHORYLASE-RXN Definition: Catalysis of the reaction: 1,4-beta-D-glucosyl(n) + phosphate = 1,4-beta-D-glucosyl(n-1) + alpha-D-glucose 1-phosphate.